{
  "term_label": "odorant binding",
  "term_id": "GO:0005549",
  "gene": "UniProtKB:A6NL26",
  "gene_symbol": "OR5B21",
  "gene_name": "Olfactory receptor 5B21"
}